{
  "gene_symbol": "BIN2",
  "gene_name": "Bridging integrator 2",
  "term_id": "GO:0002102",
  "gene": "UniProtKB:Q9UBW5",
  "term_label": "podosome"
}